{
  "term_label": "plasma membrane",
  "gene_symbol": "ALDH3B2",
  "gene": "UniProtKB:P48448",
  "gene_name": "Aldehyde dehydrogenase family 3 member B2",
  "term_id": "GO:0005886"
}